{
  "gene": "UniProtKB:A5PLL7",
  "gene_symbol": "PEDS1",
  "gene_name": "Plasmanylethanolamine desaturase 1",
  "term_id": "GO:0005789",
  "term_label": "endoplasmic reticulum membrane"
}